{
  "gene_symbol": "MYOZ1",
  "gene_name": "Myozenin-1",
  "term_id": "UNKNOWN:0002",
  "gene": "UniProtKB:Q9NP98",
  "term_label": "Unknown biological process"
}